{
  "term_label": "nucleus",
  "gene_symbol": "HELT",
  "term_id": "GO:0005634",
  "gene_name": "Hairy and enhancer of split-related protein HELT",
  "gene": "UniProtKB:A6NFD8"
}